{
  "gene": "UniProtKB:Q96MC2",
  "gene_name": "Dynein regulatory complex protein 1",
  "gene_symbol": "DRC1",
  "term_id": "GO:0060285",
  "term_label": "cilium-dependent cell motility"
}